{
  "gene_symbol": "IGKV6D-41",
  "term_label": "Unknown molecular function",
  "gene": "UniProtKB:A0A0C4DH26",
  "term_id": "UNKNOWN:0001",
  "gene_name": "Probable non-functional immunoglobulin kappa variable 6D-41"
}